{
  "gene": "UniProtKB:Q9H5I1",
  "term_label": "Unknown biological process",
  "gene_name": "Histone-lysine N-methyltransferase SUV39H2",
  "gene_symbol": "SUV39H2",
  "term_id": "UNKNOWN:0002"
}